very-low-density lipoprotein particle assembly [GO:0034379] (biological process) Relationships: is_a plasma lipoprotein particle assembly [GO:0034377] Sources: GOC:BHF, GOC:mah Definition: The non-covalent aggregation and arrangement of proteins and lipids in the liver to form a very-low-density lipoprotein particle. Also known as: VLDL assembly